negative regulation of nucleotide catabolic process [GO:0030812] (biological process) Definition: Any process that stops, prevents, or reduces the frequency, rate or extent of the chemical reactions and pathways resulting in the breakdown of nucleotides. Subtypes: negative regulation of purine nucleotide catabolic process [GO:0033122] Sources: GOC:mah Relationships: is_a negative regulation of catabolic process [GO:0009895]; is a type of GO:0030811; is a type of GO:0045980; negatively regulates nucleotide catabolic process [GO:0009166] Also known as: down regulation of nucleotide catabolic process, down-regulation of nucleotide catabolic process, downregulation of nucleotide catabolic process, negative regulation of nucleotide breakdown, negative regulation of nucleotide catabolism, negative regulation of nucleotide degradation, inhibition of nucleotide catabolic process